{
  "gene_symbol": "OR6C76",
  "term_label": "plasma membrane",
  "gene": "UniProtKB:A6NM76",
  "term_id": "GO:0005886",
  "gene_name": "Olfactory receptor 6C76"
}